{
  "gene_name": "Sodium- and chloride-dependent neutral and basic amino acid transporter B(0+)",
  "gene": "UniProtKB:Q9UN76",
  "term_id": "GO:1902270",
  "term_label": "(R)-carnitine transmembrane transport",
  "gene_symbol": "SLC6A14"
}